ketone body catabolic process [GO:0046952] (biological process) Subtypes: GO:0043442 Also known as: ketolysis, ketone body breakdown, ketone body catabolism, ketone body degradation, utilization of ketone bodies Definition: The chemical reactions and pathways resulting in the breakdown of ketone bodies, any one of the three substances: acetoacetate, D-3-hydroxybutyrate (beta-hydroxybutyrate) or acetone. Ketone bodies can be used as an energy source as an alternative to glucose. Utilization of ketone bodies in peripheral tissues involves conversion of acetoacetate to acetoacetyl-CoA, which is then converted to two molecules of acetyl-CoA. Sources: ISBN:0198506732 Relationships: is a type of GO:0044282; is a type of fatty acid derivative catabolic process [GO:1901569]; is a type of ketone body metabolic process [GO:1902224]